{
  "term_id": "GO:0006357",
  "gene_name": "Krueppel-like factor 15",
  "gene": "UniProtKB:Q9UIH9",
  "term_label": "regulation of transcription by RNA polymerase II",
  "gene_symbol": "KLF15"
}